{
  "term_label": "G protein-coupled receptor activity",
  "gene_symbol": "ADGRB2",
  "gene": "UniProtKB:O60241",
  "term_id": "GO:0004930",
  "gene_name": "Adhesion G protein-coupled receptor B2"
}